{
  "gene_name": "RalA-binding protein 1",
  "gene_symbol": "RALBP1",
  "term_id": "GO:0006898",
  "term_label": "receptor-mediated endocytosis",
  "gene": "UniProtKB:Q15311"
}